{
  "gene": "UniProtKB:P29992",
  "term_label": "action potential",
  "gene_symbol": "GNA11",
  "gene_name": "Guanine nucleotide-binding protein subunit alpha-11",
  "term_id": "GO:0001508"
}